{
  "gene": "UniProtKB:Q9NWS0",
  "term_label": "box C/D snoRNP assembly",
  "gene_symbol": "PIH1D1",
  "gene_name": "PIH1 domain-containing protein 1",
  "term_id": "GO:0000492"
}